carbon monoxide sensor activity [GO:0070027] (molecular function) Also known as: carbon monoxide sensing activity Sources: GOC:ecd Relationships: is a type of molecular sensor activity [GO:0140299]; has part carbon monoxide binding [GO:0070025] Definition: Binding to and responding, e.g. by conformational change, to changes in the cellular level of carbon monoxide (CO).